{
  "gene_name": "T cell receptor alpha variable 39",
  "gene_symbol": "TRAV39",
  "term_id": "UNKNOWN:0001",
  "term_label": "Unknown molecular function",
  "gene": "UniProtKB:A0A0B4J263"
}